{
  "gene_name": "N-alpha-acetyltransferase 16, NatA auxiliary subunit",
  "term_id": "UNKNOWN:0002",
  "gene": "UniProtKB:Q6N069",
  "gene_symbol": "NAA16",
  "term_label": "Unknown biological process"
}